carbohydrate biosynthetic process [GO:0016051] (biological process) Also known as: anabolic carbohydrate metabolic process, anabolic carbohydrate metabolism, carbohydrate anabolism, carbohydrate biosynthesis, carbohydrate formation, carbohydrate synthesis Relationships: is a type of carbohydrate metabolic process [GO:0005975]; is a type of biosynthetic process [GO:0009058] Subtypes: polysaccharide biosynthetic process [GO:0000271], GO:0009312, alditol biosynthetic process [GO:0019401], GO:0019685, D-glucarate biosynthetic process [GO:0042837], D-gluconate biosynthetic process [GO:0046178], L-idonate biosynthetic process [GO:0046182], monosaccharide biosynthetic process [GO:0046364], mannosylglycerate biosynthetic process [GO:0051479] Definition: The chemical reactions and pathways resulting in the formation of carbohydrates, any of a group of organic compounds based of the general formula Cx(H2O)y. Sources: ISBN:0198506732 Regulation: regulated by regulation of carbohydrate biosynthetic process [GO:0043255]